{
  "gene": "UniProtKB:Q92546",
  "term_label": "Unknown molecular function",
  "term_id": "UNKNOWN:0001",
  "gene_name": "RAB6A-GEF complex partner protein 2",
  "gene_symbol": "RGP1"
}